{
  "gene_name": "Small proline-rich protein 2E",
  "gene_symbol": "SPRR2E",
  "term_id": "GO:0001533",
  "term_label": "cornified envelope",
  "gene": "UniProtKB:P22531"
}